{
  "gene_symbol": "RIT2",
  "term_label": "GTPase activity",
  "term_id": "GO:0003924",
  "gene": "UniProtKB:Q99578",
  "gene_name": "GTP-binding protein Rit2"
}